{
  "gene_name": "ADP-ribosylation factor 4",
  "term_label": "intracellular protein transport",
  "gene": "UniProtKB:P18085",
  "gene_symbol": "ARF4",
  "term_id": "GO:0006886"
}